{
  "gene_name": "Arfaptin-1",
  "gene_symbol": "ARFIP1",
  "gene": "UniProtKB:P53367",
  "term_id": "GO:0032588",
  "term_label": "trans-Golgi network membrane"
}